{
  "gene_symbol": "KIR2DL1",
  "term_id": "GO:0140375",
  "gene": "UniProtKB:A0A5K1VDZ0",
  "term_label": "immune receptor activity",
  "gene_name": "KIR2DL1 protein"
}